{
  "term_id": "GO:0035102",
  "gene_name": "Polycomb group RING finger protein 2",
  "gene_symbol": "PCGF2",
  "term_label": "PRC1 complex",
  "gene": "UniProtKB:P35227"
}